regulation of R8 cell spacing in compound eye [GO:0045468] (biological process) References: PMID:11880339 Sources: GOC:dph, GOC:tb Also known as: regulation of R8 spacing, R8 cell spacing in compound eye Definition: Any process that ensures that the R8 cells are selected in a precise progressive pattern so that they are evenly spaced throughout the eye disc. Subtypes: negative regulation of R8 cell spacing in compound eye [GO:0045469], positive regulation of R8 cell spacing in compound eye [GO:0045748] Relationships: is a type of pattern specification process [GO:0007389]; is a type of regulation of biological quality [GO:0065008]; is part of compound eye development [GO:0048749]